{
  "gene": "UniProtKB:Q9UKU0",
  "gene_name": "Long-chain-fatty-acid--CoA ligase 6",
  "gene_symbol": "ACSL6",
  "term_label": "long-chain fatty-acyl-CoA biosynthetic process",
  "term_id": "GO:0035338"
}